{
  "gene": "UniProtKB:Q13018",
  "gene_symbol": "PLA2R1",
  "term_label": "plasma membrane",
  "term_id": "GO:0005886",
  "gene_name": "Secretory phospholipase A2 receptor"
}